{
  "term_label": "RNA binding",
  "gene": "UniProtKB:Q12849",
  "gene_symbol": "GRSF1",
  "gene_name": "G-rich sequence factor 1",
  "term_id": "GO:0003723"
}